negative regulation of peptidyl-tyrosine autophosphorylation [GO:1900085] (biological process) Relationships: is a type of negative regulation of protein autophosphorylation [GO:0031953]; is a type of negative regulation of peptidyl-tyrosine phosphorylation [GO:0050732]; is_a regulation of peptidyl-tyrosine autophosphorylation [GO:1900084]; negatively regulates peptidyl-tyrosine autophosphorylation [GO:0038083] Sources: GOC:TermGenie, GOC:bf Also known as: down regulation of peptidyl-tyrosine autophosphorylation, down regulation of tyrosine autophosphorylation, down-regulation of peptidyl-tyrosine autophosphorylation, down-regulation of tyrosine autophosphorylation, downregulation of peptidyl-tyrosine autophosphorylation, downregulation of tyrosine autophosphorylation, negative regulation of tyrosine autophosphorylation, down regulation of receptor tyrosine kinase autophosphorylation, down-regulation of receptor tyrosine kinase autophosphorylation, downregulation of receptor tyrosine kinase autophosphorylation, inhibition of peptidyl-tyrosine autophosphorylation, inhibition of receptor tyrosine kinase autophosphorylation, inhibition of tyrosine autophosphorylation, negative regulation of receptor tyrosine kinase autophosphorylation Definition: Any process that stops, prevents or reduces the frequency, rate or extent of peptidyl-tyrosine autophosphorylation.